{
  "term_id": "UNKNOWN:0001",
  "gene_name": "Protein stum homolog",
  "gene": "UniProtKB:Q69YW2",
  "term_label": "Unknown molecular function",
  "gene_symbol": "STUM"
}